{
  "gene": "UniProtKB:Q6PI48",
  "gene_symbol": "DARS2",
  "term_label": "aspartyl-tRNA aminoacylation",
  "term_id": "GO:0006422",
  "gene_name": "Aspartate--tRNA ligase, mitochondrial"
}